{
  "term_id": "GO:0002767",
  "gene": "UniProtKB:Q14953",
  "term_label": "immune response-inhibiting cell surface receptor signaling pathway",
  "gene_symbol": "KIR2DS5",
  "gene_name": "Killer cell immunoglobulin-like receptor 2DS5"
}